{
  "gene_symbol": "THRB",
  "term_id": "GO:0000122",
  "term_label": "negative regulation of transcription by RNA polymerase II",
  "gene_name": "Thyroid hormone receptor beta",
  "gene": "UniProtKB:P10828"
}